{
  "gene": "UniProtKB:Q8N8Q3",
  "gene_symbol": "ENDOV",
  "term_label": "cytoplasm",
  "term_id": "GO:0005737",
  "gene_name": "Endonuclease V"
}